{
  "gene_name": "E3 ubiquitin-protein ligase RNF130",
  "gene_symbol": "RNF130",
  "gene": "UniProtKB:Q86XS8",
  "term_id": "GO:0061630",
  "term_label": "ubiquitin protein ligase activity"
}